{
  "gene": "UniProtKB:Q8IXT2",
  "term_id": "GO:0005634",
  "gene_name": "Doublesex- and mab-3-related transcription factor C2",
  "gene_symbol": "DMRTC2",
  "term_label": "nucleus"
}